{
  "gene_name": "Ras-related protein Rab-5B",
  "term_id": "GO:0006886",
  "gene_symbol": "RAB5B",
  "term_label": "intracellular protein transport",
  "gene": "UniProtKB:P61020"
}